histone kinase activity [GO:0035173] (MF) Subtypes: histone H1 kinase activity [GO:0140190], GO:0140995, histone H3 kinase activity [GO:0140996], histone H4 kinase activity [GO:0140997], histone H2B kinase activity [GO:0140998], histone H2AX kinase activity [GO:0141003] Sources: GOC:bf Definition: Catalysis of the transfer of a phosphate group to a histone. Relationships: is_a protein kinase activity [GO:0004672]; is a type of GO:0140993